{
  "gene": "UniProtKB:Q13683",
  "gene_name": "Integrin alpha-7",
  "term_id": "GO:0050900",
  "gene_symbol": "ITGA7",
  "term_label": "leukocyte migration"
}